{
  "gene_name": "Junctophilin-1",
  "term_id": "GO:0016529",
  "term_label": "sarcoplasmic reticulum",
  "gene": "UniProtKB:Q9HDC5",
  "gene_symbol": "JPH1"
}